{
  "gene": "UniProtKB:O00165",
  "term_id": "GO:0015629",
  "term_label": "actin cytoskeleton",
  "gene_name": "HCLS1-associated protein X-1",
  "gene_symbol": "HAX1"
}